descending aorta development [GO:0035906] (biological process) Relationships: is a type of GO:0048856; BFO_0000050 GO:0035904 Sources: GOC:bf, GOC:dgh, MA:0002571, UBERON:0001514, Wikipedia:Descending_aorta Definition: The progression of the descending aorta over time, from its initial formation to the mature structure. The descending aorta is the portion of the aorta in a two-pass circulatory system from the arch of aorta to the point where it divides into the common iliac arteries. In a two-pass circulatory system blood passes twice through the heart to supply the body once.